{
  "term_label": "erythrocyte differentiation",
  "gene_name": "CDAN1-interacting nuclease 1",
  "gene": "UniProtKB:Q9Y2V0",
  "gene_symbol": "CDIN1",
  "term_id": "GO:0030218"
}